embryonic anal fin morphogenesis [GO:0035125] (biological process) Sources: GOC:dgh Definition: The process, occurring in the embryo, by which the anatomical structures of the embryonic anal fin are generated and organized. An anal fin is an unpaired medial fin on the ventral aspect near the caudal end of a fish, which provides lateral stability while swimming. Relationships: is a type of GO:0035122; is_a anal fin morphogenesis [GO:0035144]